{
  "term_id": "GO:0050911",
  "gene": "UniProtKB:Q8NGX6",
  "term_label": "detection of chemical stimulus involved in sensory perception of smell",
  "gene_symbol": "OR10R2",
  "gene_name": "Olfactory receptor 10R2"
}